{
  "gene": "UniProtKB:Q9P0I2",
  "gene_symbol": "EMC3",
  "gene_name": "ER membrane protein complex subunit 3",
  "term_label": "EMC complex",
  "term_id": "GO:0072546"
}